{
  "term_label": "chloride channel activity",
  "term_id": "GO:0005254",
  "gene_name": "Major facilitator superfamily domain-containing protein 8",
  "gene": "UniProtKB:Q8NHS3",
  "gene_symbol": "MFSD8"
}